{
  "gene_name": "HAUS augmin-like complex subunit 1",
  "gene_symbol": "HAUS1",
  "term_id": "GO:0070652",
  "term_label": "HAUS complex",
  "gene": "UniProtKB:Q96CS2"
}